positive regulation of renal water transport [GO:2001153] (biological process) Definition: Any process that activates or increases the frequency, rate or extent of renal water transport. Sources: GOC:obol Relationships: is_a positive regulation of transport [GO:0051050]; is a type of positive regulation of multicellular organismal process [GO:0051240]; is a type of regulation of renal water transport [GO:2001151]; positively regulates renal water transport [GO:0003097]